endocytic vesicle membrane [GO:0030666] (cellular component) Relationships: is a type of cytoplasmic vesicle membrane [GO:0030659]; is a type of bounding membrane of organelle [GO:0098588]; is part of GO:0030139 Sources: GOC:mah Definition: The lipid bilayer surrounding an endocytic vesicle. Subtypes: GO:0030669, GO:0030670, peribacteroid membrane [GO:0043661]